{
  "term_label": "nucleus",
  "gene_name": "C-terminal-binding protein 2",
  "term_id": "GO:0005634",
  "gene_symbol": "CTBP2",
  "gene": "UniProtKB:P56545"
}